positive regulation of maintenance of mitotic sister chromatid cohesion, arms [GO:2000717] (biological process) Also known as: positive regulation of maintenance of mitotic sister chromatin cohesion along arms, positive regulation of maintenance of sister chromatin cohesion along arms at mitosis Relationships: is a type of positive regulation of maintenance of mitotic sister chromatid cohesion [GO:0034184]; is a type of regulation of maintenance of mitotic sister chromatid cohesion, arms [GO:2000715]; RO_0002213 GO:0071959 Sources: GOC:mah Definition: Any process that activates or increases the frequency, rate or extent of maintenance of mitotic sister chromatid cohesion along the chromosome arms.